{
  "term_label": "extracellular space",
  "term_id": "GO:0005615",
  "gene_symbol": "ANGPTL6",
  "gene_name": "Angiopoietin-related protein 6",
  "gene": "UniProtKB:Q8NI99"
}